{
  "term_id": "GO:0005886",
  "gene_symbol": "RNH1",
  "term_label": "plasma membrane",
  "gene": "UniProtKB:P13489",
  "gene_name": "Ribonuclease inhibitor"
}